methylenetetrahydrofolate reductase [NAD(P)H] activity [GO:0004489] (molecular function) Subtypes: methylenetetrahydrofolate reductase (NADH) activity [GO:0106312], methylenetetrahydrofolate reductase (NADPH) activity [GO:0106313] References: PMID:26872964 Sources: EC:1.5.1.20 Definition: Catalysis of the reaction: 5-methyltetrahydrofolate + NAD(P)+ = 5,10-methylenetetrahydrofolate + NAD(P)H + H+. Relationships: is a type of GO:0016646 Also known as: 5,10-methylenetetrahydrofolate reductase activity, 5,10-methylenetetrahydrofolic acid reductase activity, MTHFR activity, N(5),N(10)-methylenetetrahydrofolate reductase activity, N(5,10)-methylenetetrahydrofolate reductase activity, methylenetetrahydrofolate reductase activity, methylenetetrahydrofolic acid reductase activity, 5,10-methylenetetrahydrofolate reductase (FADH) activity, 5,10-methylenetetrahydrofolate reductase (FADH2) activity, 5,10-CH(2)-H(4)folate reductase activity, 5,10-CH2-H4folate reductase activity, 5,10-methylenetetrahydrofolate reductase (FADH(2)) activity, 5,10-methylenetetrahydrofolate reductase (NADPH) activity, 5,10-methylenetetrahydropteroylglutamate reductase activity, 5-methyltetrahydrofolate:(acceptor) oxidoreductase activity, 5-methyltetrahydrofolate:NAD oxidoreductase activity, 5-methyltetrahydrofolate:NAD(+) oxidoreductase activity, 5-methyltetrahydrofolate:NAD(P)+ oxidoreductase activity, 5-methyltetrahydrofolate:NAD+ oxidoreductase activity, 5-methyltetrahydrofolate:NADP(+) oxidoreductase activity, 5-methyltetrahydrofolate:NADP+ oxidoreductase activity, MetF, N5,10-methylenetetrahydrofolate reductase activity, N5,N10-methylenetetrahydrofolate reductase activity, methylenetetrahydrofolate (reduced nicotinamide adenine dinucleotide phosphate) reductase activity, methylenetetrahydrofolate (reduced riboflavin adenine dinucleotide) reductase activity, methylenetetrahydrofolate reductase (NADPH(2)) activity, methylenetetrahydrofolate reductase (NADPH2), methylenetetrahydrofolate reductase [NAD(P)H]